{
  "term_id": "UNKNOWN:0001",
  "gene": "UniProtKB:Q5JV73",
  "term_label": "Unknown molecular function",
  "gene_symbol": "FRMPD3",
  "gene_name": "FERM and PDZ domain-containing protein 3"
}